{
  "gene_symbol": "KRT87P",
  "term_id": "GO:0005615",
  "term_label": "extracellular space",
  "gene_name": "Putative keratin-87 protein",
  "gene": "UniProtKB:A6NCN2"
}